rRNA 2'-O-methylation [GO:0000451] (biological process) Definition: The addition of a methyl group to the 2'-oxygen atom of a nucleotide residue in an rRNA molecule during ribosome biogenesis. Subtypes: snoRNA guided rRNA 2'-O-methylation [GO:0000452] Relationships: is a type of rRNA methylation [GO:0031167] Sources: GOC:curators, ISBN:1555811337